{
  "term_id": "UNKNOWN:0002",
  "gene": "UniProtKB:Q6ZMV7",
  "gene_symbol": "LEKR1",
  "term_label": "Unknown biological process",
  "gene_name": "Protein LEKR1"
}